regulation of oocyte karyosome formation [GO:0120313] (biological process) Relationships: is a type of regulation of cell cycle process [GO:0010564]; is a type of regulation of chromosome organization [GO:0033044]; is a type of GO:2000241; regulates GO:0030717 Definition: Any process that modulates the frequency, rate or extent of oocyte karyosome formation, the chromosome organization process in which meiotic chromosomes in the oocyte nucleus cluster together to form a compact spherical structure called the karyosome. References: PMID:33382409 Sources: GOC:ha, GOC:krc Subtypes: negative regulation of oocyte karyosome formation [GO:0120314], positive regulation of oocyte karyosome formation [GO:0120315]